{
  "gene_name": "Epoxide hydrolase 3",
  "gene": "UniProtKB:Q9H6B9",
  "gene_symbol": "EPHX3",
  "term_id": "UNKNOWN:0002",
  "term_label": "Unknown biological process"
}